{
  "gene": "UniProtKB:Q9Y2X7",
  "gene_name": "ARF GTPase-activating protein GIT1",
  "term_id": "GO:0043005",
  "term_label": "neuron projection",
  "gene_symbol": "GIT1"
}